{
  "term_id": "UNKNOWN:0002",
  "gene": "UniProtKB:Q8N1V8",
  "gene_name": "Uncharacterized protein encoded by LINC01561",
  "term_label": "Unknown biological process",
  "gene_symbol": "LINC01561"
}